{
  "gene_name": "Muscarinic acetylcholine receptor M5",
  "term_id": "GO:0030425",
  "gene_symbol": "CHRM5",
  "gene": "UniProtKB:P08912",
  "term_label": "dendrite"
}